{
  "gene_symbol": "ATG4B",
  "term_id": "GO:0004197",
  "term_label": "cysteine-type endopeptidase activity",
  "gene": "UniProtKB:Q9Y4P1",
  "gene_name": "Cysteine protease ATG4B"
}